{
  "gene_symbol": "TRAPPC2",
  "term_label": "Unknown molecular function",
  "term_id": "UNKNOWN:0001",
  "gene_name": "Trafficking protein particle complex subunit 2",
  "gene": "UniProtKB:P0DI81"
}